{
  "gene_symbol": "CALR3",
  "gene": "UniProtKB:Q96L12",
  "term_label": "Unknown molecular function",
  "term_id": "UNKNOWN:0001",
  "gene_name": "Calreticulin-3"
}